{
  "gene_symbol": "ARL6",
  "term_id": "GO:0060271",
  "gene_name": "ADP-ribosylation factor-like protein 6",
  "gene": "UniProtKB:Q9H0F7",
  "term_label": "cilium assembly"
}